{
  "term_label": "Unknown biological process",
  "gene_name": "Serine_threonine-protein phosphatase 5",
  "gene": "UniProtKB:P53041",
  "gene_symbol": "PPP5C",
  "term_id": "UNKNOWN:0002"
}